{
  "term_id": "GO:0030507",
  "gene": "UniProtKB:Q01484",
  "gene_symbol": "ANK2",
  "term_label": "spectrin binding",
  "gene_name": "Ankyrin-2"
}